{
  "gene_symbol": "DRD2",
  "term_id": "GO:0004930",
  "term_label": "G protein-coupled receptor activity",
  "gene": "UniProtKB:P14416",
  "gene_name": "D(2) dopamine receptor"
}